{
  "term_label": "angiogenesis",
  "term_id": "GO:0001525",
  "gene_symbol": "AMOTL1",
  "gene": "UniProtKB:Q8IY63",
  "gene_name": "Angiomotin-like protein 1"
}